{
  "gene_symbol": "TERF2IP",
  "term_id": "GO:0031848",
  "gene": "UniProtKB:Q9NYB0",
  "term_label": "protection from non-homologous end joining at telomere",
  "gene_name": "Telomeric repeat-binding factor 2-interacting protein 1"
}